ubiquitin-like protein binding [GO:0032182] (molecular function) Definition: Binding to a small conjugating protein such as ubiquitin or a ubiquitin-like protein. Also known as: small conjugating protein binding Subtypes: GO:0032183, ubiquitin binding [GO:0043130] Relationships: is a type of protein binding [GO:0005515] Sources: GOC:mah